UDP-3-dehydro-alpha-D-glucose dehydrogenase activity [GO:0102982] (molecular function) Definition: Catalysis of the reaction: UDP-alpha-D-glucose + NAD = H+ + UDP-3-keto-alpha-D-glucose + NADH. Relationships: is a type of GO:0016616 References: PMID:11278540 Sources: GOC:pz